regulation of cellular response to oxidopamine [GO:1905846] (biological process) References: PMID:23721876 Sources: GOC:TermGenie, GO_REF:0000058 Definition: Any process that modulates the frequency, rate or extent of cellular response to oxidopamine. Relationships: is_a regulation of response to stimulus [GO:0048583]; is a type of regulation of cellular process [GO:0050794]; regulates cellular response to oxidopamine [GO:1905842] Subtypes: GO:1905847, positive regulation of cellular response to oxidopamine [GO:1905848]